{
  "gene_name": "Interleukin-17 receptor E",
  "term_label": "Unknown biological process",
  "term_id": "UNKNOWN:0002",
  "gene_symbol": "IL17RE",
  "gene": "UniProtKB:Q8NFR9"
}